N-acetylneuraminate synthase activity [GO:0050462] (molecular function) Sources: EC:2.5.1.56, MetaCyc:N-ACETYLNEURAMINATE-SYNTHASE-RXN Relationships: is a type of transferase activity, transferring alkyl or aryl (other than methyl) groups [GO:0016765] Also known as: (NANA)condensing enzyme activity, N-acetylneuraminate pyruvate-lyase (pyruvate-phosphorylating) activity, N-acetylneuraminic acid synthase activity, NeuAc synthase activity, phosphoenolpyruvate:N-acetyl-D-mannosamine C-(1-carboxyvinyl)transferase (phosphate-hydrolysing, 2-carboxy-2-oxoethyl-forming) Definition: Catalysis of the reaction: phosphoenolpyruvate + N-acetyl-D-mannosamine + H2O = phosphate + N-acetylneuraminate.